maintenance of protein location in T cell secretory granule [GO:0033377] (biological process) Sources: GOC:dph, GOC:mah, GOC:tb Subtypes: maintenance of protease location in T cell secretory granule [GO:0033379] Relationships: is_a maintenance of protein location in cell [GO:0032507]; is part of GO:0033374 Also known as: maintenance of protein localization in T lymphocyte secretory granule, maintenance of protein localization in T-cell secretory granule, maintenance of protein localization in T-lymphocyte secretory granule, maintenance of protein localization in T cell secretory granule Definition: A process in which a protein is maintained in a secretory granule in a T cell and prevented from moving elsewhere.